{
  "gene_symbol": "C16orf90",
  "term_id": "UNKNOWN:0001",
  "gene_name": "Uncharacterized protein C16orf90",
  "gene": "UniProtKB:A8MZG2",
  "term_label": "Unknown molecular function"
}